hydroxymethylglutaryl-CoA reductase (NADH) activity [GO:0140643] (MF) Definition: Catalysis of the reaction: (R)-mevalonate + CoA + 2 NAD+ = 3-hydroxy-3-methylglutaryl-CoA + 2 NADH. References: PMID:29224355 Sources: RHEA:14833 Also known as: 3-hydroxy-3-methylglutaryl coenzyme A reductase activity, HMG-CoA reductase activity, beta-hydroxy-beta-methylglutaryl CoA-reductase activity, beta-hydroxy-beta-methylglutaryl coenzyme A reductase activity, hydroxymethylglutaryl coenzyme A reductase activity Note: Note that this activity is not present in eukaryotes, see PMID:29224355. Relationships: is a type of GO:0016616